{
  "term_id": "GO:0030280",
  "gene_symbol": "KRT74",
  "gene": "UniProtKB:Q7RTS7",
  "term_label": "structural constituent of skin epidermis",
  "gene_name": "Keratin, type II cytoskeletal 74"
}